{
  "gene_name": "Tissue factor pathway inhibitor",
  "gene_symbol": "TFPI",
  "gene": "UniProtKB:P10646",
  "term_label": "Unknown biological process",
  "term_id": "UNKNOWN:0002"
}